{
  "term_label": "Unknown biological process",
  "gene": "UniProtKB:Q9C073",
  "gene_symbol": "FAM117A",
  "gene_name": "Protein FAM117A",
  "term_id": "UNKNOWN:0002"
}